{
  "term_id": "UNKNOWN:0001",
  "gene_name": "Ubiquitin carboxyl-terminal hydrolase 33",
  "gene": "UniProtKB:Q8TEY7",
  "gene_symbol": "USP33",
  "term_label": "Unknown molecular function"
}